{
  "term_label": "actin filament binding",
  "gene_symbol": "FLII",
  "term_id": "GO:0051015",
  "gene": "UniProtKB:Q13045",
  "gene_name": "Protein flightless-1 homolog"
}